AP-1 adaptor complex [GO:0030121] (cellular component) Relationships: is a type of clathrin adaptor complex [GO:0030131]; is part of clathrin coat of trans-Golgi network vesicle [GO:0030130] Also known as: HA1, HA1 clathrin adaptor, AP-1 related adapter complex Definition: A heterotetrameric AP-type membrane coat adaptor complex that consists of beta1, gamma, mu1 and sigma1 subunits and links clathrin to the membrane surface of a vesicle; vesicles with AP-1-containing coats are normally found primarily in the trans-Golgi network. In at least humans, the AP-1 complex can be heterogeneric due to the existence of multiple subunit isoforms encoded by different genes (gamma1 and gamma2, mu1A and mu1B, and sigma1A, sigma1B and sigma1C). References: PMID:10611976, PMID:21097499 Sources: GOC:mah